{
  "gene": "UniProtKB:Q658Y4",
  "gene_name": "Protein FAM91A1",
  "gene_symbol": "FAM91A1",
  "term_label": "trans-Golgi network",
  "term_id": "GO:0005802"
}